{
  "gene_name": "Adenosine 3'-phospho 5'-phosphosulfate transporter 1",
  "gene_symbol": "SLC35B2",
  "term_label": "endoplasmic reticulum membrane",
  "gene": "UniProtKB:Q8TB61",
  "term_id": "GO:0005789"
}